{
  "term_id": "UNKNOWN:0003",
  "gene": "UniProtKB:Q4V321",
  "gene_name": "G antigen 13",
  "gene_symbol": "GAGE13",
  "term_label": "Unknown cellular component"
}